{
  "term_id": "GO:0015722",
  "term_label": "canalicular bile acid transport",
  "gene_name": "Bile salt export pump",
  "gene_symbol": "ABCB11",
  "gene": "UniProtKB:O95342"
}